regulation of lysosomal protein catabolic process [GO:1905165] (biological process) Definition: Any process that modulates the frequency, rate or extent of lysosomal protein catabolic process. Also known as: regulation of cellular protein breakdown in lysosome, regulation of cellular protein catabolic process in lysosome, regulation of cellular protein catabolism in lysosome, regulation of cellular protein degradation in lysosome, regulation of lysosomal protein catabolism, regulation of lysosomal protein degradation, regulation of lysosomal proteolysis, regulation of proteolysis within lysosome Subtypes: negative regulation of lysosomal protein catabolic process [GO:1905166], positive regulation of lysosomal protein catabolic process [GO:1905167] Relationships: is a type of regulation of protein catabolic process in the vacuole [GO:1904350]; regulates lysosomal protein catabolic process [GO:1905146] References: PMID:23499937 Sources: GOC:PARL, GOC:TermGenie, GOC:bf, GO_REF:0000058